{
  "gene": "UniProtKB:A8MYP8",
  "term_label": "cytoskeleton",
  "gene_symbol": "CIMAP1B",
  "term_id": "GO:0005856",
  "gene_name": "Outer dense fiber protein 3B"
}